indoleacetic acid conjugate biosynthetic process [GO:0033474] (biological process) Definition: The chemical reactions and pathways resulting in the formation of an indole-3-acetic acid conjugate, a form of indoleacetic acid covalently bound to another molecule. Relationships: is a type of auxin biosynthetic process [GO:0009851]; is a type of indoleacetic acid conjugate metabolic process [GO:0033473]; is a type of indole-containing compound biosynthetic process [GO:0042435] Also known as: IAA conjugate biosynthetic process, indole acetic acid conjugate biosynthesis, indole acetic acid conjugate biosynthetic process, indoleacetic acid conjugate anabolism, indoleacetic acid conjugate biosynthesis, indoleacetic acid conjugate formation, indoleacetic acid conjugate synthesis Subtypes: indoleacetic acid amide conjugate biosynthetic process [GO:0033475], GO:0033476 Sources: GOC:mah